{
  "term_id": "GO:0055038",
  "gene_symbol": "EHD3",
  "gene_name": "EH domain-containing protein 3",
  "gene": "UniProtKB:Q9NZN3",
  "term_label": "recycling endosome membrane"
}